nitric oxide reductase [NAD(P)H] activity [GO:0102199] (molecular function) Sources: EC:1.7.1.14 Relationships: is a type of oxidoreductase activity, acting on other nitrogenous compounds as donors, with NAD or NADP as acceptor [GO:0046857] Definition: Catalysis of the reaction: H2O + NAD(P)+ + nitrous oxide = H+ + NAD(P)H + 2 nitric oxide. Also known as: nitric oxide reductase activity (NAD(P)H-dependent) activity